{
  "term_id": "GO:1902600",
  "gene_name": "Sodium_potassium-transporting ATPase subunit alpha-4",
  "gene_symbol": "ATP1A4",
  "gene": "UniProtKB:Q13733",
  "term_label": "proton transmembrane transport"
}